synapse assembly [GO:0007416] (biological process) Regulation: regulated by regulation of synapse assembly [GO:0051963]; negatively regulated by GO:0051964; positively regulated by positive regulation of synapse assembly [GO:0051965] Also known as: synapse biogenesis, synaptogenesis Sources: GOC:mah Relationships: is a type of cell junction assembly [GO:0034329]; is a type of GO:0050808; is part of nervous system development [GO:0007399] Subtypes: synaptic assembly at neuromuscular junction [GO:0051124], GO:0060386, GO:1904861, inhibitory synapse assembly [GO:1904862] Definition: The aggregation, arrangement and bonding together of a set of components to form a synapse. This process ends when the synapse is mature (functional).